positive regulation of cardiac muscle hypertrophy in response to stress [GO:1903244] (biological process) References: PMID:19287093 Sources: GOC:BHF, GOC:TermGenie, GOC:rl, GO_REF:0000058 Relationships: is a type of positive regulation of cardiac muscle hypertrophy [GO:0010613]; is a type of GO:0010615; is a type of regulation of cardiac muscle hypertrophy in response to stress [GO:1903242]; RO_0002213 cardiac muscle hypertrophy in response to stress [GO:0014898] Also known as: up regulation of cardiac muscle hypertrophy in response to stress, up-regulation of cardiac muscle hypertrophy in response to stress, upregulation of cardiac muscle hypertrophy in response to stress, activation of cardiac muscle hypertrophy in response to stress Definition: Any process that activates or increases the frequency, rate or extent of cardiac muscle hypertrophy in response to stress.